{
  "gene_symbol": "GLT1D1",
  "gene": "UniProtKB:Q96MS3",
  "term_id": "UNKNOWN:0003",
  "gene_name": "Glycosyltransferase 1 domain-containing protein 1",
  "term_label": "Unknown cellular component"
}